salutaridine reductase (NADPH) activity [GO:0047037] (molecular function) Also known as: salutaridinol:NADP+ 7-oxidoreductase activity Relationships: is a type of oxidoreductase activity, acting on the CH-OH group of donors, NAD or NADP as acceptor [GO:0016616] Definition: Catalysis of the reaction: (7S)-salutaridinol + NADP+ = H+ + NADPH + salutaridine. Sources: EC:1.1.1.248, RHEA:10108